{
  "gene_symbol": "C7orf31",
  "term_label": "centrosome",
  "term_id": "GO:0005813",
  "gene": "UniProtKB:Q8N865",
  "gene_name": "Uncharacterized protein C7orf31"
}